{
  "gene_name": "Prenylcysteine oxidase-like",
  "gene_symbol": "PCYOX1L",
  "term_id": "GO:0030327",
  "term_label": "prenylated protein catabolic process",
  "gene": "UniProtKB:Q8NBM8"
}